{
  "gene": "UniProtKB:Q5TZJ5",
  "term_id": "UNKNOWN:0001",
  "gene_name": "Spermatogenesis-associated protein 31A1",
  "gene_symbol": "SPATA31A1",
  "term_label": "Unknown molecular function"
}